cytoplasmic microtubule [GO:0005881] (cellular component) Sources: GOC:mah Relationships: is a type of microtubule [GO:0005874]; is part of GO:0005737 Subtypes: astral microtubule [GO:0000235], axonemal microtubule [GO:0005879], GO:0055028 Definition: Any microtubule in the cytoplasm of a cell. Also known as: non-spindle-associated astral microtubule